{
  "gene_symbol": "HRNR",
  "gene_name": "Hornerin",
  "gene": "UniProtKB:Q86YZ3",
  "term_label": "cornified envelope",
  "term_id": "GO:0001533"
}